{
  "gene_name": "Prickle-like protein 4",
  "gene": "UniProtKB:Q2TBC4",
  "gene_symbol": "PRICKLE4",
  "term_label": "adherens junction",
  "term_id": "GO:0005912"
}